{
  "gene_name": "Actin filament-associated protein 1-like 1",
  "gene_symbol": "AFAP1L1",
  "gene": "UniProtKB:Q8TED9",
  "term_id": "UNKNOWN:0002",
  "term_label": "Unknown biological process"
}